{
  "term_label": "regulation of DNA-templated transcription",
  "gene_symbol": "ZNF280B",
  "term_id": "GO:0006355",
  "gene": "UniProtKB:Q86YH2",
  "gene_name": "Zinc finger protein 280B"
}